{
  "gene_name": "Adenosine receptor A2b",
  "gene": "UniProtKB:P29275",
  "gene_symbol": "ADORA2B",
  "term_label": "G protein-coupled adenosine receptor activity",
  "term_id": "GO:0001609"
}